lysine racemase activity [GO:0018113] (molecular function) Sources: EC:5.1.1.5 Definition: Catalysis of the reaction: L-lysine = D-lysine. Relationships: is a type of amino-acid racemase activity [GO:0047661]